{
  "term_id": "GO:0043065",
  "gene_symbol": "LATS1",
  "gene_name": "Serine_threonine-protein kinase LATS1",
  "gene": "UniProtKB:O95835",
  "term_label": "positive regulation of apoptotic process"
}